{
  "gene_name": "Heat shock transcription factor, X-linked member 3",
  "gene": "UniProtKB:A0A1B0GWH4",
  "term_label": "DNA-binding transcription factor activity",
  "term_id": "GO:0003700",
  "gene_symbol": "HSFX3"
}